meiotic cell cycle phase [GO:0098762] (biological process) Definition: One of the distinct periods or stages into which the meiotic cell cycle is divided. Each phase is characterized by the occurrence of specific biochemical and morphological events. Sources: GOC:dos Relationships: is a type of cell cycle phase [GO:0022403]; happens during meiotic cell cycle [GO:0051321] Subtypes: GO:0051323, meiotic M phase [GO:0051327], meiotic interphase [GO:0051328], GO:0098764, GO:0098765 Note: This term should not be used for direct annotation. If you are trying to make an annotation to x phase, it is likely that the correct annotation should be to 'regulation of x/y phase transition' or to a process which occurs during the reported phase (e.g. mitotic DNA replication for mitotic S-phase). To capture the phase when a specific location or process is observed, the phase term can be used in an annotation extension (PMID:24885854) applied to a cellular component term (with the relation exists_during) or a biological process term (with the relation happens_during).